{
  "gene": "UniProtKB:Q13467",
  "gene_symbol": "FZD5",
  "gene_name": "Frizzled-5",
  "term_label": "non-canonical Wnt signaling pathway",
  "term_id": "GO:0035567"
}